prospore membrane leading edge [GO:0070056] (cellular component) References: PMID:14702385 Sources: GOC:mah Relationships: is a type of GO:0016020; is part of prospore membrane [GO:0005628] Definition: The region of the prospore membrane that extends to surround the spore nucleus; coated with specific proteins that are thought to play a role in prospore membrane organization. Also known as: forespore membrane leading edge